regulation of adenylate cyclase-inhibiting adrenergic receptor signaling pathway [GO:0071877] (biological process) Definition: Any process that modulates the frequency, rate or extent of an adenylate cyclase-inhibiting adrenergic receptor signaling pathway activity. An adrenergic receptor signaling pathway is the series of molecular signals generated as a consequence of an adrenergic receptor binding to one of its physiological ligands. Sources: GOC:BHF, GOC:mah Also known as: regulation of adrenergic receptor signaling pathway, regulation of adrenergic receptor signalling pathway Relationships: is a type of GO:0008277; regulates adenylate cyclase-inhibiting adrenergic receptor signaling pathway [GO:0071881]